{
  "term_id": "GO:0005516",
  "gene_name": "IQ domain-containing protein F2",
  "gene": "UniProtKB:Q8IXL9",
  "gene_symbol": "IQCF2",
  "term_label": "calmodulin binding"
}